ATP-dependent protein folding chaperone [GO:0140662] (molecular function) Definition: Binding to a protein or a protein-containing complex to assist the protein folding process, driven by ATP hydrolysis. References: PMID:27365453 Relationships: is a type of protein folding chaperone [GO:0044183]; is a type of GO:0140657